nucleoside-triphosphate-hexose-1-phosphate nucleotidyltransferase activity [GO:0047339] (molecular function) Relationships: is a type of GO:0016779 Sources: EC:2.7.7.28, MetaCyc:2.7.7.28-RXN Also known as: NDP-hexose diphosphorylase activity, NDP-hexose pyrophosphorylase activity, GDP hexose pyrophosphorylase activity, GTP:alpha-D-hexose-1-phosphate guanylyltransferase activity, GTP:hexose-1-phosphate guanylyltransferase activity, guanosine diphosphohexose pyrophosphorylase activity, hexose-1-phosphate guanylyltransferase activity, NDP hexose pyrophosphorylase activity, NTP:alpha-D-aldose-1-phosphate nucleotidyltransferase activity, NTP:hexose-1-phosphate nucleotidyltransferase activity, hexose 1-phosphate guanylyltransferase activity, hexose 1-phosphate nucleotidyltransferase activity, hexose nucleotidylating enzyme activity, nucleoside diphosphohexose pyrophosphorylase activity, nucleoside-triphosphate-aldose-1-phosphate nucleotidyltransferase activity Definition: Catalysis of the reaction: hexose 1-phosphate + nucleoside triphosphate = NDP-hexose + diphosphate.